{
  "term_id": "UNKNOWN:0001",
  "gene": "UniProtKB:Q71F56",
  "gene_symbol": "MED13L",
  "term_label": "Unknown molecular function",
  "gene_name": "Mediator of RNA polymerase II transcription subunit 13-like"
}